{
  "gene_name": "Dual specificity testis-specific protein kinase 2",
  "term_label": "nucleus",
  "term_id": "GO:0005634",
  "gene": "UniProtKB:Q96S53",
  "gene_symbol": "TESK2"
}